{
  "gene_symbol": "TTLL8",
  "term_label": "sperm flagellum",
  "gene": "UniProtKB:A6PVC2",
  "gene_name": "Protein monoglycylase TTLL8",
  "term_id": "GO:0036126"
}